{
  "term_label": "Unknown molecular function",
  "term_id": "UNKNOWN:0001",
  "gene_name": "phospholipase A2 inhibitor and Ly6_PLAUR domain-containing protein",
  "gene_symbol": "PINLYP",
  "gene": "UniProtKB:A6NC86"
}